{
  "term_id": "GO:0036435",
  "gene": "UniProtKB:Q96EP0",
  "gene_name": "E3 ubiquitin-protein ligase RNF31",
  "gene_symbol": "RNF31",
  "term_label": "K48-linked polyubiquitin modification-dependent protein binding"
}